{
  "term_label": "chloride channel activity",
  "term_id": "GO:0005254",
  "gene_name": "Glycine receptor subunit alpha-3",
  "gene_symbol": "GLRA3",
  "gene": "UniProtKB:O75311"
}